(S)-2-(5-amino-1-(5-phospho-D-ribosyl)imidazole-4-carboxamido) succinate lyase (fumarate-forming) activity [GO:0070626] (molecular function) Relationships: is a type of amidine-lyase activity [GO:0016842] Sources: RHEA:23920 Definition: Catalysis of the reaction: (S)-2-(5-amino-1-(5-phospho-D-ribosyl)imidazole-4-carboxamido)succinate = fumarate + 5-amino-1-(5-phospho-D-ribosyl)imidazole-4-carboxamide. Also known as: adenylosuccinase activity, adenylosuccinate lyase activity, succino AMP-lyase activity, (S)-2-(5-amino-1-(5-phospho-D-ribosyl)imidazole-4-carboxamido)succinate AMP-lyase (fumarate-forming) activity, SAICAR-lyase (fumarate forming) activity